beta-glucogallin O-galloyltransferase activity [GO:0047201] (molecular function) Sources: EC:2.3.1.90, RHEA:11416 Definition: Catalysis of the reaction: 2 1-O-galloyl-beta-D-glucose = 1,6-bis-O-galloyl-beta-D-glucose + D-glucose. Relationships: is a type of acyltransferase activity, transferring groups other than amino-acyl groups [GO:0016747] Also known as: 1-O-galloyl-beta-D-glucose:1-O-galloyl-beta-D-glucose O-galloyltransferase activity